{
  "gene_symbol": "KCND2",
  "gene_name": "Potassium voltage-gated channel subfamily D member 2",
  "gene": "UniProtKB:Q9NZV8",
  "term_id": "GO:0001508",
  "term_label": "action potential"
}